{
  "gene": "UniProtKB:Q49AG3",
  "term_id": "UNKNOWN:0003",
  "term_label": "Unknown cellular component",
  "gene_name": "Zinc finger BED domain-containing protein 5",
  "gene_symbol": "ZBED5"
}